{
  "term_label": "positive regulation of insulin secretion",
  "gene": "UniProtKB:Q86V21",
  "gene_name": "Acetoacetyl-CoA synthetase",
  "gene_symbol": "AACS",
  "term_id": "GO:0032024"
}